{
  "gene": "UniProtKB:Q9BZE9",
  "gene_name": "Tether containing UBX domain for GLUT4",
  "term_id": "GO:0006886",
  "gene_symbol": "ASPSCR1",
  "term_label": "intracellular protein transport"
}